{
  "term_label": "Unknown molecular function",
  "term_id": "UNKNOWN:0001",
  "gene_symbol": "CBLN1",
  "gene_name": "Cerebellin-1",
  "gene": "UniProtKB:P23435"
}